{
  "term_id": "GO:0003796",
  "gene": "UniProtKB:Q96QH8",
  "term_label": "lysozyme activity",
  "gene_symbol": "SPACA5",
  "gene_name": "Sperm acrosome-associated protein 5"
}